{
  "gene_symbol": "ULBP2",
  "term_label": "antigen processing and presentation of endogenous peptide antigen via MHC class I via ER pathway, TAP-independent",
  "term_id": "GO:0002486",
  "gene_name": "UL16-binding protein 2",
  "gene": "UniProtKB:Q9BZM5"
}